positive regulation of granulocyte colony-stimulating factor production [GO:0071657] (biological process) Also known as: positive regulation of CSF3 production, positive regulation of G-CSF production, positive regulation of colony stimulating factor 3 (granulocyte) production, positive regulation of filgrastim production, positive regulation of granulocyte colony stimulating factor production, positive regulation of lenograstim production, positive regulation of pluripoietin production Sources: GOC:mah Definition: Any process that activates or increases the frequency, rate, or extent of production of granulocyte colony-stimulating factor. Relationships: is a type of regulation of granulocyte colony-stimulating factor production [GO:0071655]; is a type of positive regulation of macrophage colony-stimulating factor production [GO:1901258]; positively regulates granulocyte colony-stimulating factor production [GO:0071611]